{
  "gene_symbol": "OVGP1",
  "term_label": "extracellular region",
  "term_id": "GO:0005576",
  "gene": "UniProtKB:Q12889",
  "gene_name": "Oviduct-specific glycoprotein"
}